regulation of post-translational protein targeting to membrane, translocation [GO:0120235] (biological process) Also known as: regulation of posttranslational endoplasmic reticulum membrane protein translocation, regulation of posttranslational protein targeting to membrane, translocation, regulation of N-terminal signal peptide-independent translocation into the ER, regulation of SRP-independent endoplasmic reticulum protein-membrane targeting, translocation Definition: Any process that modulates the frequency, rate or extent of posttranslational protein translocation through the ER membrane. References: PMID:32513868 Sources: GOC:krc, GOC:rn Subtypes: negative regulation of post-translational protein targeting to membrane, translocation [GO:0120236] Relationships: is_a regulation of intracellular protein transport [GO:0033157]; is a type of regulation of transmembrane transport [GO:0034762]; regulates post-translational protein targeting to membrane, translocation [GO:0031204]